mitomycin C catabolic process [GO:1901776] (biological process) Also known as: mitomycin C breakdown, mitomycin C catabolism, mitomycin C degradation Relationships: is a type of ketone catabolic process [GO:0042182] References: PMID:10094699, PMID:10099135 Sources: GOC:TermGenie, GOC:yaf Definition: The chemical reactions and pathways resulting in the breakdown of mitomycin C.